regulation of larval somatic muscle development [GO:0062229] (biological process) Definition: Any process that modulates the rate, frequency or extent of larval somatic muscle development. References: PMID:16643882, PMID:25758712 Relationships: is a type of regulation of somatic muscle development [GO:0062223]; regulates larval somatic muscle development [GO:0007526] Subtypes: GO:0062230, positive regulation of larval somatic muscle development [GO:0062231]